5'-acylphosphoadenosine hydrolase activity [GO:0047586] (molecular function) Relationships: is a type of hydrolase activity, acting on acid anhydrides, in phosphorus-containing anhydrides [GO:0016818] Sources: EC:3.6.1.20, MetaCyc:5-ACYLPHOSPHOADENOSINE-HYDROLASE-RXN Also known as: 5'-acylphosphoadenosine acylhydrolase activity, 5-phosphoadenosine hydrolase activity Definition: Catalysis of the reaction: 5'-acylphosphoadenosine + H2O = AMP + a carboxylate.